{
  "gene": "UniProtKB:P46379",
  "term_label": "misfolded protein binding",
  "gene_symbol": "BAG6",
  "term_id": "GO:0051787",
  "gene_name": "Large proline-rich protein BAG6"
}